positive regulation of interleukin-32 production [GO:0150191] (BP) Sources: GOC:aruk Also known as: positive regulation of interleukin-32 biosynthetic process, positive regulation of interleukin-32 secretion Relationships: is a type of GO:0001819; is a type of GO:0150189; positively regulates interleukin-32 production [GO:0072637] Definition: Any process that activates or increases the frequency, rate or extent of interleukin-32 production.